CD27 signaling pathway [GO:0160162] (biological process) Relationships: is a type of cell surface receptor signaling pathway [GO:0007166] Definition: The series of molecular signals initiated by the binding of the cell surface receptor CD27 to its physiological ligand CD70, and ending with the regulation of a downstream cellular process, e.g. transcription. References: PMID:26359318, PMID:8387892